kinetochore microtubule [GO:0005828] (cellular component) Subtypes: mitotic spindle kinetochore microtubule [GO:1990941] Sources: ISBN:0815316194 Relationships: is_a spindle microtubule [GO:0005876] Definition: Any of the spindle microtubules that attach to the kinetochores of chromosomes by their plus ends, and maneuver the chromosomes during mitotic or meiotic chromosome segregation. Also known as: pole-to-kinetochore microtubule